{
  "gene_symbol": "INSL3",
  "term_label": "Unknown molecular function",
  "gene": "UniProtKB:P51460",
  "gene_name": "Insulin-like 3",
  "term_id": "UNKNOWN:0001"
}